{
  "gene": "UniProtKB:P10746",
  "gene_name": "Uroporphyrinogen-III synthase",
  "term_id": "GO:0005829",
  "term_label": "cytosol",
  "gene_symbol": "Mgu"
}